{
  "gene": "UniProtKB:P05067",
  "gene_symbol": "APP",
  "term_label": "cell surface",
  "term_id": "GO:0009986",
  "gene_name": "Amyloid-beta precursor protein"
}